lead ion transport [GO:0015692] (biological process) Relationships: is a type of metal ion transport [GO:0030001] Sources: GOC:ai Definition: The directed movement of lead (Pb) ions into, out of or within a cell, or between cells, by means of some agent such as a transporter or pore.